{
  "term_label": "nucleus",
  "gene": "UniProtKB:Q06455",
  "gene_symbol": "RUNX1T1",
  "gene_name": "Protein CBFA2T1",
  "term_id": "GO:0005634"
}